{
  "gene_symbol": "WNT4",
  "term_label": "canonical Wnt signaling pathway",
  "gene": "UniProtKB:P56705",
  "gene_name": "Protein Wnt-4",
  "term_id": "GO:0060070"
}